betaine aldehyde catabolic process [GO:1902062] (biological process) References: PMID:23563483 Sources: GOC:TermGenie, GOC:di Definition: The chemical reactions and pathways resulting in the breakdown of betaine aldehyde. Also known as: betaine aldehyde breakdown, betaine aldehyde catabolism, betaine aldehyde degradation Relationships: is_a GO:0009056